{
  "gene_name": "Olfactory receptor 51Q1",
  "term_label": "plasma membrane",
  "gene_symbol": "OR51Q1",
  "gene": "UniProtKB:Q8NH59",
  "term_id": "GO:0005886"
}